{
  "term_id": "GO:0043491",
  "gene_symbol": "NYAP1",
  "gene_name": "Neuronal tyrosine-phosphorylated phosphoinositide-3-kinase adapter 1",
  "term_label": "phosphatidylinositol 3-kinase/protein kinase B signal transduction",
  "gene": "UniProtKB:Q6ZVC0"
}